{
  "gene_name": "Low-density lipoprotein receptor",
  "term_label": "lipoprotein particle binding",
  "term_id": "GO:0071813",
  "gene_symbol": "LDLR",
  "gene": "UniProtKB:P01130"
}